{
  "gene_symbol": "SNRPN",
  "gene_name": "Small nuclear ribonucleoprotein-associated protein N",
  "term_label": "U2-type prespliceosome",
  "gene": "UniProtKB:P63162",
  "term_id": "GO:0071004"
}